{
  "term_id": "UNKNOWN:0001",
  "gene_symbol": "D2HGDH",
  "gene": "UniProtKB:Q8N465",
  "gene_name": "D-2-hydroxyglutarate dehydrogenase, mitochondrial",
  "term_label": "Unknown molecular function"
}